{
  "gene_name": "Syntabulin",
  "gene": "UniProtKB:Q9NX95",
  "gene_symbol": "SYBU",
  "term_id": "GO:0005881",
  "term_label": "cytoplasmic microtubule"
}